{
  "gene_name": "Annexin A2",
  "gene_symbol": "ANXA2",
  "term_label": "calcium-dependent phospholipid binding",
  "term_id": "GO:0005544",
  "gene": "UniProtKB:P07355"
}